positive regulation of nuclear migration along microtubule [GO:1902840] (biological process) Relationships: is_a positive regulation of intracellular transport [GO:0032388]; is a type of regulation of nuclear migration along microtubule [GO:1902838]; positively regulates GO:0030473 References: PMID:23087209 Sources: GOC:TermGenie, GO_REF:0000058 Definition: Any process that activates or increases the frequency, rate or extent of nuclear migration along microtubule. Also known as: positive regulation of microtubule cytoskeleton-dependent nuclear positioning, positive regulation of microtubule cytoskeleton-dependent nucleus positioning, positive regulation of microtubule-dependent nuclear positioning, positive regulation of microtubule-dependent nucleus positioning, positive regulation of microtubule-mediated nuclear migration, positive regulation of nuclear migration, microtubule-mediated, positive regulation of transport of nucleus by microtubules, positive regulation of transport of nucleus, microtubule-mediated, up regulation of microtubule cytoskeleton-dependent nuclear positioning, up regulation of microtubule cytoskeleton-dependent nucleus positioning, up regulation of microtubule-dependent nuclear positioning, up regulation of microtubule-dependent nucleus positioning, up regulation of microtubule-mediated nuclear migration, up regulation of nuclear migration along microtubule, up regulation of nuclear migration, microtubule-mediated, up regulation of transport of nucleus by microtubules, up regulation of transport of nucleus, microtubule-mediated, up-regulation of microtubule cytoskeleton-dependent nuclear positioning, up-regulation of microtubule cytoskeleton-dependent nucleus positioning, up-regulation of microtubule-dependent nuclear positioning, up-regulation of microtubule-dependent nucleus positioning, up-regulation of microtubule-mediated nuclear migration, up-regulation of nuclear migration along microtubule, up-regulation of nuclear migration, microtubule-mediated, up-regulation of transport of nucleus by microtubules, up-regulation of transport of nucleus, microtubule-mediated, upregulation of microtubule cytoskeleton-dependent nuclear positioning, upregulation of microtubule cytoskeleton-dependent nucleus positioning, upregulation of microtubule-dependent nuclear positioning, upregulation of microtubule-dependent nucleus positioning, upregulation of microtubule-mediated nuclear migration, upregulation of nuclear migration along microtubule, upregulation of nuclear migration, microtubule-mediated, upregulation of transport of nucleus by microtubules, upregulation of transport of nucleus, microtubule-mediated, activation of microtubule cytoskeleton-dependent nuclear positioning, activation of microtubule cytoskeleton-dependent nucleus positioning, activation of microtubule-dependent nuclear positioning, activation of microtubule-dependent nucleus positioning, activation of microtubule-mediated nuclear migration, activation of nuclear migration along microtubule, activation of nuclear migration, microtubule-mediated, activation of transport of nucleus by microtubules, activation of transport of nucleus, microtubule-mediated Subtypes: positive regulation of nuclear migration during mitotic telophase [GO:1902854]